neural tube closure [GO:0001843] (BP) Relationships: is a type of tube closure [GO:0060606]; is part of primary neural tube formation [GO:0014020] Definition: The last step in the formation of the neural tube, where the paired neural folds are brought together and fuse at the dorsal midline. Sources: GOC:dph, ISBN:0878932437